metanephric cap formation [GO:0072187] (BP) Sources: GOC:mtg_kidney_jan10 Subtypes: metanephric cap specification [GO:0072188] Definition: The developmental process pertaining to the initial formation of a metanephric cap from unspecified parts. The metanephric cap is formed by the condensation of metanephric mesenchymal cells surrounding the ureteric bud tip. Relationships: is a type of anatomical structure formation involved in morphogenesis [GO:0048646]; BFO_0000050 metanephric cap morphogenesis [GO:0072186]